{
  "gene": "UniProtKB:Q9Y2R9",
  "gene_name": "Small ribosomal subunit protein uS7m",
  "term_id": "GO:0003729",
  "term_label": "mRNA binding",
  "gene_symbol": "MRPS7"
}